{
  "gene": "UniProtKB:Q12965",
  "gene_symbol": "MYO1E",
  "gene_name": "Unconventional myosin-Ie",
  "term_label": "actin filament organization",
  "term_id": "GO:0007015"
}